{
  "gene_symbol": "TRAV12-1",
  "gene": "UniProtKB:A0A0B4J245",
  "term_label": "peptide antigen binding",
  "gene_name": "T cell receptor alpha variable 12-1",
  "term_id": "GO:0042605"
}